{
  "gene": "UniProtKB:Q6PKH6",
  "gene_name": "Dehydrogenase_reductase SDR family member 4-like 2",
  "term_label": "peroxisome",
  "gene_symbol": "DHRS4L2",
  "term_id": "GO:0005777"
}